alkaloid metabolic process [GO:0009820] (biological process) Relationships: is a type of metabolic process [GO:0008152] Sources: GOC:lr, ISBN:0122146743 Also known as: alkaloid metabolism Definition: The chemical reactions and pathways involving alkaloids, nitrogen containing natural products which are not otherwise classified as peptides, nonprotein amino acids, amines, cyanogenic glycosides, glucosinolates, cofactors, phytohormones or primary metabolites (such as purine or pyrimidine bases). Subtypes: nicotinamide metabolic process [GO:0006769], alkaloid biosynthetic process [GO:0009821], alkaloid catabolic process [GO:0009822], isoquinoline alkaloid metabolic process [GO:0033076], GO:0035834, purine alkaloid metabolic process [GO:0046446], nicotinate metabolic process [GO:1901847]